purine nucleoside interconversion [GO:0019686] (biological process) Relationships: is a type of GO:0015949; is a type of purine nucleoside metabolic process [GO:0042278] Subtypes: GO:0019688 Sources: GOC:mah, ISBN:0306444747, ISBN:0471394831 Definition: The chemical reactions and pathways by which a purine nucleoside is synthesized from another purine nucleoside.